{
  "term_id": "GO:0005829",
  "term_label": "cytosol",
  "gene_name": "Ribokinase",
  "gene_symbol": "RBKS",
  "gene": "UniProtKB:Q9H477"
}